{
  "gene": "UniProtKB:Q7Z3Z4",
  "term_label": "piRNA binding",
  "term_id": "GO:0034584",
  "gene_symbol": "PIWIL4",
  "gene_name": "Piwi-like protein 4"
}